 [go#goslim:agr] Note: AGR slim